embryonic hemocyte differentiation [GO:0035163] (biological process) References: PMID:14602069 Sources: GOC:bf, GOC:mtg_sensu Also known as: embryonic arthropod blood cell differentiation, embryonic hemocyte cell differentiation Relationships: is_a GO:0042386; is part of embryonic hemopoiesis [GO:0035162] Subtypes: GO:0035164, GO:0035165 Definition: The process in which a relatively unspecialized cell derived from the embryonic head mesoderm acquires the specialized features of a mature hemocyte. Hemocytes are blood cells associated with a hemocoel (the cavity containing most of the major organs of the arthropod body) which are involved in defense and clotting of hemolymph, but not involved in transport of oxygen.